protocadherin-alpha-v7-protocadherin-gamma-b2 complex [GO:0071190] (cellular component) Also known as: Pcdha7-Pcdhgb4 complex Relationships: is_a GO:0071183 Definition: A protein complex that contains the cell adhesion molecules protocadherin-alpha-v7 and protocadherin-gamma-b2, and is involved in the regulation of protein localization to the plasma membrane. References: PMID:15347688